{
  "term_label": "Unknown molecular function",
  "gene_symbol": "SBSPON",
  "gene": "UniProtKB:Q8IVN8",
  "gene_name": "Somatomedin-B and thrombospondin type-1 domain-containing protein",
  "term_id": "UNKNOWN:0001"
}